{
  "gene": "UniProtKB:A8MY62",
  "term_id": "UNKNOWN:0002",
  "gene_symbol": "LACTBL1",
  "gene_name": "Putative beta-lactamase-like 1",
  "term_label": "Unknown biological process"
}